chromosome separation [GO:0051304] (biological process) Regulation: regulated by regulation of chromosome separation [GO:1905818]; negatively regulated by negative regulation of chromosome separation [GO:1905819]; positively regulated by GO:1905820 Subtypes: mitotic sister chromatid separation [GO:0051306], meiotic chromosome separation [GO:0051307] References: PMID:20352243 Sources: GOC:ai, GOC:lb, GOC:mah, GOC:mtg_cell_cycle Definition: The cell cycle process in which paired chromosomes are detached from each other. Chromosome separation begins with the release of cohesin complexes from chromosomes; in budding yeast, this includes the cleavage of cohesin complexes along the chromosome arms, followed by the separation of the centromeric regions. Chromosome separation also includes formation of chromatid axes mediated by condensins, and ends with the disentangling of inter-sister catenation catalyzed by topoisomerase II (topo II). Also known as: rDNA separation, chromatid release Relationships: is a type of cell cycle process [GO:0022402]; is part of chromosome segregation [GO:0007059]